ribonuclease D activity [GO:0033890] (molecular function) Sources: EC:3.1.13.5 Relationships: is a type of RNA exonuclease activity, producing 5'-phosphomonoesters [GO:0016896] Definition: Catalysis of the exonucleolytic cleavage that removes extra residues from the 3'-terminus of tRNA to produce 5'-mononucleotides. Also known as: RNase D activity